{
  "term_id": "GO:0006614",
  "term_label": "SRP-dependent cotranslational protein targeting to membrane",
  "gene": "UniProtKB:O76094",
  "gene_name": "Signal recognition particle subunit SRP72",
  "gene_symbol": "SRP72"
}